{
  "gene_name": "Rho-related GTP-binding protein RhoN",
  "term_id": "GO:0005525",
  "gene": "UniProtKB:P52198",
  "gene_symbol": "RND2",
  "term_label": "GTP binding"
}